{
  "gene": "UniProtKB:Q5T7N2",
  "term_label": "single-stranded RNA binding",
  "term_id": "GO:0003727",
  "gene_symbol": "L1TD1",
  "gene_name": "LINE-1 type transposase domain-containing protein 1"
}